{
  "gene_name": "Gastrokine-3",
  "gene_symbol": "GKN3P",
  "term_label": "extracellular space",
  "term_id": "GO:0005615",
  "gene": "UniProtKB:P0CG01"
}